{
  "term_label": "sensory organ development",
  "term_id": "GO:0007423",
  "gene_name": "Paired box protein Pax-8",
  "gene": "UniProtKB:Q06710",
  "gene_symbol": "PAX8"
}